{
  "gene_symbol": "H2BC20P",
  "term_id": "GO:0003677",
  "gene": "UniProtKB:Q6DN03",
  "gene_name": "Putative histone H2B type 2-C",
  "term_label": "DNA binding"
}